oxalate metabolic process [GO:0033609] (biological process) Also known as: ethanedioate metabolic process, ethanedioic acid metabolic process, oxalate metabolism, oxalic acid metabolic process Subtypes: oxalate biosynthetic process [GO:0033610], oxalate catabolic process [GO:0033611] Definition: The chemical reactions and pathways involving oxalate, the organic acid ethanedioate. Sources: GOC:mlg Relationships: is a type of GO:0043648